response to hypochlorite [GO:1901530] (BP) Definition: Any process that results in a change in state or activity of a cell or an organism (in terms of movement, secretion, enzyme production, gene expression, etc.) as a result of a hypochlorite stimulus. Relationships: is a type of response to reactive oxygen species [GO:0000302] References: PMID:22223481 Sources: GOC:TermGenie, GOC:pr